{
  "gene_symbol": "IL5RA",
  "gene": "UniProtKB:Q01344",
  "gene_name": "Interleukin-5 receptor subunit alpha",
  "term_id": "GO:0008284",
  "term_label": "positive regulation of cell population proliferation"
}